regulation of membrane repolarization during cardiac muscle cell action potential [GO:1905031] (BP) Definition: Any process that modulates the frequency, rate or extent of membrane repolarization during cardiac muscle cell action potential. Relationships: is a type of regulation of membrane repolarization during action potential [GO:0098903]; is_a regulation of cardiac muscle cell membrane repolarization [GO:0099623]; regulates membrane repolarization during cardiac muscle cell action potential [GO:0086013] Subtypes: regulation of membrane repolarization during atrial cardiac muscle cell action potential [GO:1905000], regulation of membrane repolarization during ventricular cardiac muscle cell action potential [GO:1905024], GO:1905032, positive regulation of membrane repolarization during cardiac muscle cell action potential [GO:1905033] References: PMID:23157812 Sources: GOC:BHF, GOC:BHF_miRNA, GOC:TermGenie, GOC:mtg_cardiac_conduct_nov11, GOC:rph